{
  "gene": "UniProtKB:P08133",
  "term_id": "GO:0001786",
  "gene_symbol": "ANXA6",
  "term_label": "phosphatidylserine binding",
  "gene_name": "Annexin A6"
}